{
  "gene_name": "Large ribosomal subunit protein uL1m",
  "term_label": "structural constituent of ribosome",
  "gene": "UniProtKB:Q9BYD6",
  "term_id": "GO:0003735",
  "gene_symbol": "MRPL1"
}